{
  "gene": "UniProtKB:P03971",
  "gene_name": "Muellerian-inhibiting factor",
  "term_label": "gonad development",
  "gene_symbol": "AMH",
  "term_id": "GO:0008406"
}